{
  "gene_symbol": "PNLDC1",
  "gene_name": "Poly(A)-specific ribonuclease PNLDC1",
  "term_label": "siRNA 3'-end processing",
  "term_id": "GO:1990432",
  "gene": "UniProtKB:Q8NA58"
}